phenylacetate-CoA ligase activity [GO:0047475] (molecular function) Relationships: is a type of CoA-ligase activity [GO:0016405]; is_a acid-thiol ligase activity [GO:0016878] Definition: Catalysis of the reaction: ATP + CoA + phenylacetate = AMP + diphosphate + H+ + phenylacetyl-CoA. Sources: RHEA:20956 Also known as: PA-CoA ligase activity, phenacyl coenzyme A synthetase activity, phenylacetate:CoA ligase (AMP-forming), phenylacetyl-CoA ligase (AMP-forming), phenylacetyl-CoA ligase activity